{
  "term_label": "DNA-binding transcription factor activity, RNA polymerase II-specific",
  "term_id": "GO:0000981",
  "gene_symbol": "ZFP1",
  "gene_name": "Zinc finger protein 1 homolog",
  "gene": "UniProtKB:Q6P2D0"
}